{
  "term_label": "Unknown molecular function",
  "gene": "UniProtKB:A6NKW6",
  "term_id": "UNKNOWN:0001",
  "gene_name": "Protein shisa-like-2B",
  "gene_symbol": "SHISAL2B"
}